{
  "term_id": "GO:0007420",
  "term_label": "brain development",
  "gene": "UniProtKB:Q04741",
  "gene_symbol": "EMX1",
  "gene_name": "Homeobox protein EMX1"
}